{
  "gene_symbol": "CIB1",
  "gene_name": "Calcium and integrin-binding protein 1",
  "term_id": "GO:0005737",
  "term_label": "cytoplasm",
  "gene": "UniProtKB:Q99828"
}